negative regulation of emericellamide A biosynthetic process [GO:1900662] (biological process) Relationships: is a type of negative regulation of emericellamide biosynthetic process [GO:1900659]; is a type of regulation of emericellamide A biosynthetic process [GO:1900661]; RO_0002212 GO:1900617 Also known as: down regulation of emericellamide A anabolism, down regulation of emericellamide A biosynthesis, down regulation of emericellamide A biosynthetic process, down regulation of emericellamide A formation, down regulation of emericellamide A synthesis, down-regulation of emericellamide A anabolism, down-regulation of emericellamide A biosynthesis, down-regulation of emericellamide A biosynthetic process, down-regulation of emericellamide A formation, down-regulation of emericellamide A synthesis, downregulation of emericellamide A anabolism, downregulation of emericellamide A biosynthesis, downregulation of emericellamide A biosynthetic process, downregulation of emericellamide A formation, downregulation of emericellamide A synthesis, inhibition of emericellamide A anabolism, inhibition of emericellamide A biosynthesis, inhibition of emericellamide A formation, inhibition of emericellamide A synthesis, negative regulation of emericellamide A anabolism, negative regulation of emericellamide A biosynthesis, negative regulation of emericellamide A formation, negative regulation of emericellamide A synthesis, inhibition of emericellamide A biosynthetic process Definition: Any process that stops, prevents or reduces the frequency, rate or extent of emericellamide A biosynthetic process. Sources: GOC:TermGenie, GOC:di